{
  "term_id": "GO:0035591",
  "gene_name": "Adapter molecule crk",
  "term_label": "signaling adaptor activity",
  "gene": "UniProtKB:P46108",
  "gene_symbol": "CRK"
}